{
  "gene_symbol": "TYW1",
  "gene_name": "S-adenosyl-L-methionine-dependent tRNA 4-demethylwyosine synthase TYW1",
  "term_label": "Unknown cellular component",
  "gene": "UniProtKB:Q9NV66",
  "term_id": "UNKNOWN:0003"
}